(S)-hydroxynitrile lyase activity [GO:0047606] (molecular function) Definition: Catalysis of the reaction: a (S)-hydroxynitrile = hydrogen cyanide + an aldehyde or ketone. References: PMID:3377504 Sources: EC:4.1.2.47 Also known as: hydroxynitrilase activity, hydroxynitrile lyase activity, alpha-hydroxynitrile lyase activity, oxynitrilase activity Subtypes: aliphatic (S)-hydroxynitrile lyase activity [GO:0052891], aromatic (S)-hydroxynitrile lyase activity [GO:0052892] Relationships: is_a aldehyde-lyase activity [GO:0016832]